{
  "term_id": "UNKNOWN:0003",
  "gene": "UniProtKB:P0DJD8",
  "gene_symbol": "PGA3",
  "term_label": "Unknown cellular component",
  "gene_name": "Pepsin A-3"
}